{
  "term_label": "cytosol",
  "gene_name": "RAF proto-oncogene serine_threonine-protein kinase",
  "gene": "UniProtKB:P04049",
  "gene_symbol": "RAF1",
  "term_id": "GO:0005829"
}